chorion-containing eggshell formation [GO:0007304] (BP) Definition: The construction of a chorion-containing eggshell. An example of this is found in Drosophila melanogaster. Also known as: eggshell formation Relationships: is a type of eggshell formation [GO:0030703]; is part of follicle cell of egg chamber development [GO:0030707]; has part egg chorion assembly [GO:0007306] Sources: GOC:mah, GOC:mtg_sensu